{
  "term_label": "chemokine activity",
  "gene_symbol": "CCL1",
  "term_id": "GO:0008009",
  "gene": "UniProtKB:P22362",
  "gene_name": "C-C motif chemokine 1"
}